{
  "term_label": "ubiquitin protein ligase activity",
  "gene_name": "Tripartite motif-containing protein 54",
  "gene_symbol": "TRIM54",
  "term_id": "GO:0061630",
  "gene": "UniProtKB:Q9BYV2"
}